fibrous ring of heart morphogenesis [GO:1905285] (biological process) References: PMID:16037571 Sources: GOC:BHF, GOC:TermGenie, GOC:rl, GO_REF:0000083 Relationships: is a type of tissue morphogenesis [GO:0048729] Definition: The developmental process by which a fibrous ring of heart is generated and organized. Also known as: anulus fibrosus of heart morphogenesis, Lower's ring morphogenesis, annulus fibrosus cordis morphogenesis, anulus fibrosus cordis morphogenesis, aortic annulus morphogenesis, atrioventricular ring morphogenesis, coronary tendon morphogenesis